antigen sampling by M cells in mucosal-associated lymphoid tissue [GO:0002406] (biological process) Definition: The process of antigen samples carried out by M cells in the mucosal-associated lymphoid tissue. Also known as: antigen sampling by M cells in MALT References: PMID:11896763 Sources: GOC:jal Relationships: is a type of antigen sampling in mucosal-associated lymphoid tissue [GO:0002404]